{
  "gene": "UniProtKB:A0A1B0GUV7",
  "term_label": "Unknown biological process",
  "term_id": "UNKNOWN:0002",
  "gene_name": "Testis-expressed protein 48",
  "gene_symbol": "TEX48"
}